{
  "gene": "UniProtKB:Q6IB77",
  "gene_symbol": "GLYAT",
  "gene_name": "Glycine N-acyltransferase",
  "term_label": "mitochondrion",
  "term_id": "GO:0005739"
}